cell migration [GO:0016477] (biological process) Definition: The controlled self-propelled movement of a cell from one site to a destination guided by molecular cues. Sources: GOC:cjm, GOC:dph, GOC:ems, GOC:pf, Wikipedia:Cell_migration Relationships: is a type of GO:0048870 Subtypes: ameboidal-type cell migration [GO:0001667], GO:0001764, hepatocyte cell migration [GO:0002194], GO:0003428, substrate-dependent cell migration [GO:0006929], dorsal closure, spreading of leading edge cells [GO:0007395], glial cell migration [GO:0008347], germ cell migration [GO:0008354], muscle cell migration [GO:0014812], cell migration in hindbrain [GO:0021535], hypothalamus cell migration [GO:0021855], forebrain cell migration [GO:0021885], hemocyte migration [GO:0035099], cell migration involved in vasculogenesis [GO:0035441], angioblast cell migration [GO:0035476], hematopoietic stem cell migration [GO:0035701], cell migration involved in kidney development [GO:0035787], GO:0040039, endothelial cell migration [GO:0043542], wound healing, spreading of cells [GO:0044319], neuromast primordium migration [GO:0048883], leukocyte migration [GO:0050900], cell chemotaxis [GO:0060326], cell migration involved in heart development [GO:0060973], GO:0061334, GO:0061457, GO:0090248, neuroblast migration [GO:0097402], lymphoid lineage cell migration [GO:0097534], distal tip cell migration [GO:0097628], sperm migration through the uterotubal junction [GO:0160131], GO:1902766, anterior visceral endoderm cell migration [GO:1905070], mesenchymal stem cell migration [GO:1905319], pericyte cell migration [GO:1905351] Regulation: RO_0002211 by regulation of cell migration [GO:0030334]; positively regulated by GO:0030335; negatively regulated by GO:0030336